{
  "gene_name": "26S proteasome non-ATPase regulatory subunit 7",
  "gene_symbol": "PSMD7",
  "gene": "UniProtKB:P51665",
  "term_label": "proteasome-mediated ubiquitin-dependent protein catabolic process",
  "term_id": "GO:0043161"
}